{
  "gene": "UniProtKB:O95907",
  "gene_symbol": "SLC16A8",
  "term_id": "GO:0016323",
  "term_label": "basolateral plasma membrane",
  "gene_name": "Monocarboxylate transporter 3"
}